fatty acid beta-oxidation, unsaturated, odd number [GO:0033541] (biological process) Sources: GOC:mah, MetaCyc:PWY-5137 Relationships: is a type of GO:0006635 Definition: A fatty acid beta-oxidation pathway by which fatty acids having cis-double bonds on odd-numbered carbons are degraded. In this pathway, a cis-3-enoyl-CoA is generated by the core beta-oxidation pathway, and then converted to a trans-2-enoyl-CoA, which can return to the core beta-oxidation pathway for complete degradation. Fatty acid beta-oxidation begins with the addition of coenzyme A to a fatty acid, and ends when only two or three carbons remain (as acetyl-CoA or propionyl-CoA respectively).